{
  "gene_symbol": "CD244",
  "gene_name": "Natural killer cell receptor 2B4",
  "term_id": "GO:0006955",
  "term_label": "immune response",
  "gene": "UniProtKB:Q9BZW8"
}